{
  "term_id": "UNKNOWN:0001",
  "gene": "UniProtKB:O75487",
  "term_label": "Unknown molecular function",
  "gene_symbol": "GPC4",
  "gene_name": "Glypican-4"
}